{
  "gene_symbol": "USP29",
  "gene": "UniProtKB:Q9HBJ7",
  "term_label": "nucleus",
  "term_id": "GO:0005634",
  "gene_name": "Ubiquitin carboxyl-terminal hydrolase 29"
}